detection of muramyl dipeptide [GO:0032498] (biological process) Relationships: is a type of GO:0032495; is a type of detection of peptidoglycan [GO:0032499] References: PMID:15998797 Sources: GOC:rl Definition: The series of events in which a muramyl dipeptide stimulus is received by a cell and converted into a molecular signal. Muramyl dipeptide is derived from peptidoglycan.